regulation of gamma-delta T cell proliferation [GO:0046646] (BP) Also known as: regulation of gamma-delta T lymphocyte proliferation, regulation of gamma-delta T-cell proliferation, regulation of gamma-delta T-lymphocyte proliferation Sources: GOC:ai Definition: Any process that modulates the frequency, rate or extent of gamma-delta T cell proliferation. Relationships: is a type of regulation of T cell proliferation [GO:0042129]; is a type of regulation of gamma-delta T cell activation [GO:0046643]; regulates GO:0046630 Subtypes: negative regulation of gamma-delta T cell proliferation [GO:0046647], positive regulation of gamma-delta T cell proliferation [GO:0046648]